memory B cell differentiation [GO:0002319] (biological process) Sources: GOC:jal, ISBN:0781735149 Note: Note that immunologists typically use the word 'development' to refer to cells of B or T cell lineages undergoing the process that GO describes as 'cell differentiation'. Also known as: memory B lymphocyte differentiation, memory B-cell differentiation, memory B-lymphocyte differentiation, memory B cell development Relationships: is a type of mature B cell differentiation involved in immune response [GO:0002313]; is a type of GO:0090715 Definition: The process in which a B cell acquires the specialized features of a memory B cell. Memory B cells are cells that can respond rapidly to antigen re-exposure by production of high-affinity antibody.